phytanate-CoA ligase activity [GO:0050197] (molecular function) Relationships: is a type of CoA-ligase activity [GO:0016405]; is a type of GO:0016878 Definition: Catalysis of the reaction: ATP + CoA + phytanate = AMP + diphosphate + H+ + phytanoyl-CoA. Sources: EC:6.2.1.24, RHEA:21380 Also known as: phytanate:CoA ligase (AMP-forming), phytanoyl-CoA ligase activity